{
  "term_id": "GO:0008593",
  "gene": "UniProtKB:Q9H488",
  "gene_name": "GDP-fucose protein O-fucosyltransferase 1",
  "term_label": "regulation of Notch signaling pathway",
  "gene_symbol": "POFUT1"
}